{
  "gene": "UniProtKB:P51810",
  "term_label": "plasma membrane",
  "gene_symbol": "GPR143",
  "gene_name": "G-protein coupled receptor 143",
  "term_id": "GO:0005886"
}